{
  "term_label": "Unknown molecular function",
  "gene": "UniProtKB:Q9BWD3",
  "gene_name": "Retrotransposon Gag-like protein 8A",
  "gene_symbol": "RTL8A",
  "term_id": "UNKNOWN:0001"
}